kidney rudiment formation [GO:0072003] (biological process) Definition: The developmental process pertaining to the initial formation of a kidney rudiment from unspecified parts. A kidney is an organ that filters the blood and excretes the end products of body metabolism in the form of urine. Sources: GOC:mtg_kidney_jan10 Also known as: kidney anlage formation Relationships: is a type of anatomical structure formation involved in morphogenesis [GO:0048646]; is part of GO:0060993 Subtypes: pronephros formation [GO:0072116]